{
  "term_label": "RNA polymerase I core promoter sequence-specific DNA binding",
  "gene_name": "TATA box-binding protein-associated factor RNA polymerase I subunit C",
  "gene_symbol": "TAF1C",
  "term_id": "GO:0001164",
  "gene": "UniProtKB:Q15572"
}